{
  "gene": "UniProtKB:O95479",
  "gene_name": "GDH_6PGL endoplasmic bifunctional protein",
  "gene_symbol": "H6PD",
  "term_id": "GO:0009051",
  "term_label": "pentose-phosphate shunt, oxidative branch"
}